{
  "term_label": "Unknown cellular component",
  "term_id": "UNKNOWN:0003",
  "gene_name": "Protein SOGA3",
  "gene": "UniProtKB:Q5TF21",
  "gene_symbol": "SOGA3"
}